{
  "gene_symbol": "N4BP2",
  "gene": "UniProtKB:Q86UW6",
  "term_label": "endonuclease activity",
  "term_id": "GO:0004519",
  "gene_name": "NEDD4-binding protein 2"
}